{
  "gene_name": "Survival motor neuron protein",
  "gene_symbol": "SMN2",
  "gene": "UniProtKB:Q16637",
  "term_id": "GO:0032797",
  "term_label": "SMN complex"
}